{
  "term_label": "cytosol",
  "term_id": "GO:0005829",
  "gene_name": "Transforming acidic coiled-coil-containing protein 1",
  "gene_symbol": "TACC1",
  "gene": "UniProtKB:O75410"
}